{
  "gene_name": "HLA class II histocompatibility antigen, DM alpha chain",
  "term_id": "GO:0005765",
  "gene": "UniProtKB:P28067",
  "gene_symbol": "HLA-DMA",
  "term_label": "lysosomal membrane"
}